{
  "term_label": "Unknown cellular component",
  "gene_symbol": "HLX",
  "term_id": "UNKNOWN:0003",
  "gene_name": "H2.0-like homeobox protein",
  "gene": "UniProtKB:Q14774"
}